{
  "gene": "UniProtKB:P51693",
  "gene_symbol": "APLP1",
  "term_label": "central nervous system development",
  "gene_name": "Amyloid beta precursor like protein 1",
  "term_id": "GO:0007417"
}